{
  "gene_name": "Olfactory receptor 5L1",
  "gene_symbol": "OR5L1",
  "term_label": "Unknown cellular component",
  "term_id": "UNKNOWN:0003",
  "gene": "UniProtKB:Q8NGL2"
}